antigen processing and presentation of lipid antigen via MHC class Ib [GO:0048003] (biological process) Regulation: regulated by regulation of antigen processing and presentation of lipid antigen via MHC class Ib [GO:0002598]; RO_0002212 by negative regulation of antigen processing and presentation of lipid antigen via MHC class Ib [GO:0002599]; positively regulated by GO:0002600 Definition: The process in which an antigen-presenting cell expresses lipid antigen in association with an MHC class Ib protein complex on its cell surface, including lipid extraction, degradation, and transport steps for the lipid antigen both prior to and following assembly with the MHC protein complex. The lipid antigen may originate from an endogenous or exogenous source of lipid. Class Ib here refers to non-classical class I molecules, such as those of the CD1 family. Subtypes: antigen processing and presentation, endogenous lipid antigen via MHC class Ib [GO:0048006], antigen processing and presentation, exogenous lipid antigen via MHC class Ib [GO:0048007] Also known as: antigen presentation, lipid antigen, lipid antigen processing and presentation via MHC class Ib Relationships: is a type of GO:0002475 References: PMID:10375559, PMID:15928678, PMID:15928680 Sources: GOC:add